{
  "term_label": "cilium assembly",
  "gene_symbol": "TEKT3",
  "gene_name": "Tektin-3",
  "gene": "UniProtKB:Q9BXF9",
  "term_id": "GO:0060271"
}